{
  "term_id": "GO:0007157",
  "gene_symbol": "CD6",
  "gene": "UniProtKB:P30203",
  "term_label": "heterophilic cell-cell adhesion",
  "gene_name": "T-cell differentiation antigen CD6"
}